{
  "gene_symbol": "KRBOX1",
  "term_id": "GO:0005634",
  "gene_name": "KRAB domain-containing protein 1",
  "term_label": "nucleus",
  "gene": "UniProtKB:C9JBD0"
}